alcohol dehydrogenase [NAD(P)+] activity [GO:0018455] (molecular function) Also known as: alcohol:NAD(P)+ oxidoreductase activity, aldehyde reductase (NADPH/NADH) Subtypes: alcohol dehydrogenase (NAD+) activity [GO:0004022], GO:0008106, 3-methylbutanal reductase [NAD(P)H] activity [GO:0046568] Definition: Catalysis of the reaction: an alcohol + NAD(P)+ = an aldehyde or ketone + NAD(P)H + H+. Sources: GOC:curators Relationships: is a type of oxidoreductase activity, acting on the CH-OH group of donors, NAD or NADP as acceptor [GO:0016616]